serotonin receptor activity [GO:0099589] (MF) Sources: GOC:dos Relationships: is a type of transmembrane signaling receptor activity [GO:0004888] Subtypes: serotonin-gated monoatomic cation channel activity [GO:0022850], serotonin-gated chloride channel activity [GO:0160039] Definition: Combining with the biogenic amine serotonin and transmitting a signal across a membrane by activating some effector activity. Serotonin (5-hydroxytryptamine) is a neurotransmitter and hormone found in vertebrates and invertebrates.